{
  "gene": "UniProtKB:Q15582",
  "gene_name": "Transforming growth factor-beta-induced protein ig-h3",
  "term_id": "GO:0050839",
  "term_label": "cell adhesion molecule binding",
  "gene_symbol": "TGFBI"
}